{
  "gene_name": "Putative PRAME family member 26",
  "gene": "UniProtKB:H0Y7S4",
  "gene_symbol": "PRAMEF26",
  "term_label": "proteasome-mediated ubiquitin-dependent protein catabolic process",
  "term_id": "GO:0043161"
}